{
  "gene_symbol": "SLC2A4RG",
  "term_id": "GO:0003700",
  "gene": "UniProtKB:Q9NR83",
  "term_label": "DNA-binding transcription factor activity",
  "gene_name": "SLC2A4 regulator"
}